KICSTOR complex [GO:0140007] (cellular component) References: PMID:28199306 Definition: A protein complex that regulates the TORC1 signaling pathway in response to nutrients. The KICSTOR complex is composed of KPTN, ITFG2, C12orf66 and SZT2. Relationships: is a type of GO:0032991